{
  "term_id": "GO:0010468",
  "term_label": "regulation of gene expression",
  "gene_symbol": "ZNF711",
  "gene": "UniProtKB:Q9Y462",
  "gene_name": "Zinc finger protein 711"
}